{
  "gene_symbol": "DLG3",
  "term_id": "GO:0097120",
  "term_label": "receptor localization to synapse",
  "gene": "UniProtKB:Q92796",
  "gene_name": "Disks large homolog 3"
}